{
  "gene_symbol": "OR6B2",
  "term_id": "GO:0005549",
  "gene_name": "Olfactory receptor 6B2",
  "term_label": "odorant binding",
  "gene": "UniProtKB:Q6IFH4"
}